positive regulation of tissue remodeling [GO:0034105] (BP) Relationships: is a type of regulation of tissue remodeling [GO:0034103]; is a type of positive regulation of multicellular organismal process [GO:0051240]; positively regulates tissue remodeling [GO:0048771] Sources: GOC:add Subtypes: positive regulation of erythrocyte clearance [GO:0034108], positive regulation of bone remodeling [GO:0046852], positive regulation of mammary gland involution [GO:1903521], positive regulation of connective tissue replacement [GO:1905205], positive regulation of blood vessel remodeling [GO:2000504] Definition: Any process that activates or increases the frequency, rate, or extent of tissue remodeling. Also known as: positive regulation of tissue remodelling